{
  "gene": "UniProtKB:P12272",
  "term_id": "UNKNOWN:0003",
  "gene_symbol": "PTHLH",
  "gene_name": "Parathyroid hormone-related protein",
  "term_label": "Unknown cellular component"
}